{
  "term_label": "mRNA 3'-UTR binding",
  "gene": "UniProtKB:Q32P51",
  "term_id": "GO:0003730",
  "gene_name": "Heterogeneous nuclear ribonucleoprotein A1-like 2",
  "gene_symbol": "HNRNPA1L2"
}